{
  "gene_symbol": "DLGAP3",
  "gene_name": "Disks large-associated protein 3",
  "gene": "UniProtKB:O95886",
  "term_label": "modulation of chemical synaptic transmission",
  "term_id": "GO:0050804"
}